{
  "gene": "UniProtKB:Q9UHC6",
  "gene_name": "Contactin-associated protein-like 2",
  "term_id": "GO:0007612",
  "gene_symbol": "CNTNAP2",
  "term_label": "learning"
}